{
  "gene_symbol": "DOC2A",
  "gene_name": "Double C2-like domain-containing protein alpha",
  "term_id": "GO:0098850",
  "term_label": "extrinsic component of synaptic vesicle membrane",
  "gene": "UniProtKB:Q14183"
}